{
  "gene": "UniProtKB:Q9H4M9",
  "gene_name": "EH domain-containing protein 1",
  "gene_symbol": "EHD1",
  "term_id": "GO:0005737",
  "term_label": "cytoplasm"
}